{
  "term_label": "Unknown cellular component",
  "term_id": "UNKNOWN:0003",
  "gene": "UniProtKB:Q9H1I8",
  "gene_symbol": "ASCC2",
  "gene_name": "Activating signal cointegrator 1 complex subunit 2"
}